{
  "term_id": "UNKNOWN:0003",
  "term_label": "Unknown cellular component",
  "gene_name": "Ubiquitin-conjugating enzyme E2 R1",
  "gene": "UniProtKB:P49427",
  "gene_symbol": "CDC34"
}